{
  "term_id": "UNKNOWN:0003",
  "gene_name": "Epididymal protein 13",
  "term_label": "Unknown cellular component",
  "gene_symbol": "EDDM13",
  "gene": "UniProtKB:A0A1B0GTR0"
}